{
  "term_label": "Unknown molecular function",
  "term_id": "UNKNOWN:0001",
  "gene": "UniProtKB:Q8N865",
  "gene_name": "Uncharacterized protein C7orf31",
  "gene_symbol": "C7orf31"
}